regulation of peptidyl-lysine crotonylation [GO:0120093] (biological process) Subtypes: negative regulation of peptidyl-lysine crotonylation [GO:0120094] Definition: Any process that modulates the frequency, rate or extent of crotonylation of a lysine residue in a protein. Relationships: is a type of GO:0031399; regulates peptidyl-lysine crotonylation [GO:0140066] References: PMID:28803779